{
  "term_label": "transcription coregulator activity",
  "gene_symbol": "TCERG1",
  "gene": "UniProtKB:O14776",
  "term_id": "GO:0003712",
  "gene_name": "Transcription elongation regulator 1"
}